{
  "term_id": "GO:0006357",
  "gene_name": "Zinc finger protein 705D",
  "gene_symbol": "ZNF705D",
  "term_label": "regulation of transcription by RNA polymerase II",
  "gene": "UniProtKB:P0CH99"
}